{
  "term_label": "mitophagy",
  "gene": "UniProtKB:Q14457",
  "term_id": "GO:0000423",
  "gene_name": "Beclin-1",
  "gene_symbol": "BECN1"
}